{
  "gene_name": "PRAME family member 1",
  "term_id": "GO:0043161",
  "term_label": "proteasome-mediated ubiquitin-dependent protein catabolic process",
  "gene": "UniProtKB:O95521",
  "gene_symbol": "PRAMEF1"
}